positive regulation of adenosine receptor signaling pathway [GO:0060168] (BP) Relationships: is a type of positive regulation of G protein-coupled receptor signaling pathway [GO:0045745]; is a type of GO:0060167; RO_0002213 GO:0001973 Sources: GOC:dph Definition: Any process that activates or increases the frequency, rate or extent of the adenosine receptor signaling pathway. The adenosine receptor pathway is the series of molecular signals generated as a consequence of an adenosine receptor binding to one of its physiological ligands. Also known as: positive regulation of adenosine receptor signalling pathway